regulation of neuroblast migration [GO:0061853] (biological process) Subtypes: positive regulation of neuroblast migration [GO:0061854], GO:0061855 References: PMID:23149556 Definition: Any process that modulates the frequency, rate or extent of neuroblast migration. Relationships: is a type of GO:0030334; RO_0002211 GO:0097402